alpha-D-ribose 1-methylphosphonate 5-phosphate C-P-lyase activity [GO:0098848] (molecular function) Sources: EC:4.7.1.1, GOC:dos, GOC:ik Relationships: is a type of carbon phosphorus lyase activity [GO:0018835] Also known as: alpha-D-ribose-1-methylphosphonate-5-phosphate C-P-lyase (methane forming) Definition: Catalysis of the reaction: alpha-D-ribose 1-methylphosphonate 5-phosphate = alpha-D-ribose 1,2-cyclic phosphate 5-phosphate + methane.